photosystem I assembly [GO:0048564] (biological process) Definition: The aggregation, arrangement and bonding together of a set of components to form a photosystem I complex on the thylakoid membrane. Sources: GOC:go_curators Relationships: is a type of GO:0065003; is part of GO:0019684